{
  "gene_name": "Zinc finger CCHC domain-containing protein 13",
  "term_id": "GO:0045182",
  "term_label": "translation regulator activity",
  "gene_symbol": "ZCCHC13",
  "gene": "UniProtKB:Q8WW36"
}